{
  "gene": "UniProtKB:Q9P2P6",
  "term_id": "GO:0051225",
  "gene_name": "StAR-related lipid transfer protein 9",
  "term_label": "spindle assembly",
  "gene_symbol": "STARD9"
}